{
  "gene_symbol": "GATA6",
  "gene": "UniProtKB:Q92908",
  "term_id": "GO:0000978",
  "gene_name": "Transcription factor GATA-6",
  "term_label": "RNA polymerase II cis-regulatory region sequence-specific DNA binding"
}